regulation of mitochondrial transcription [GO:1903108] (biological process) Definition: Any process that modulates the frequency, rate or extent of transcription occurring in the mitochondrion. Relationships: is a type of regulation of DNA-templated transcription [GO:0006355]; is a type of regulation of mitochondrial gene expression [GO:0062125]; regulates mitochondrial transcription [GO:0006390] Subtypes: negative regulation of mitochondrial transcription [GO:0170070], positive regulation of mitochondrial transcription [GO:1903109] References: PMID:21357609 Sources: GOC:TermGenie, GO_REF:0000058 Also known as: regulation of transcription from mitochondrial promoter